{
  "term_label": "Unknown molecular function",
  "gene_name": "Protein moonraker",
  "gene": "UniProtKB:Q2KHM9",
  "term_id": "UNKNOWN:0001",
  "gene_symbol": "KIAA0753"
}